{
  "gene": "UniProtKB:P49765",
  "term_id": "GO:0060754",
  "gene_name": "Vascular endothelial growth factor B",
  "term_label": "positive regulation of mast cell chemotaxis",
  "gene_symbol": "VEGFB"
}